{
  "term_id": "GO:0001954",
  "gene_symbol": "CCL28",
  "gene_name": "C-C motif chemokine 28",
  "term_label": "positive regulation of cell-matrix adhesion",
  "gene": "UniProtKB:Q9NRJ3"
}